cellular response to pheromone [GO:0071444] (biological process) Subtypes: response to pheromone triggering conjugation with cellular fusion [GO:0000749], response to pheromone regulating conjugation with mutual genetic exchange [GO:0000756] Also known as: cellular pheromone response Sources: GOC:mah Relationships: is a type of GO:0019236; is a type of cellular response to chemical stimulus [GO:0070887] Definition: Any process that results in a change in state or activity of a cell (in terms of movement, secretion, enzyme production, gene expression, etc.) as a result of a pheromone stimulus.